fungal-type cell wall beta-glucan metabolic process [GO:0070879] (biological process) Subtypes: GO:0034408, fungal-type cell wall beta-glucan biosynthetic process [GO:0070880], fungal-type cell wall (1->3)-beta-D-glucan metabolic process [GO:0071969] Relationships: is a type of cell wall beta-glucan metabolic process [GO:0034406]; is a type of fungal-type cell wall polysaccharide metabolic process [GO:0071966]; is part of GO:0009272 Sources: GOC:mah, GOC:vw Definition: The chemical reactions and pathways involving beta-glucans, compounds composed of glucose residues linked by beta-D-glucosidic bonds, found in the walls of fungal cells. Also known as: fungal-type cell wall beta-glucan metabolism